{
  "term_label": "interleukin-10-mediated signaling pathway",
  "term_id": "GO:0140105",
  "gene": "UniProtKB:P22301",
  "gene_symbol": "IL10",
  "gene_name": "Interleukin-10"
}